{
  "gene_symbol": "DOC2A",
  "term_id": "UNKNOWN:0001",
  "term_label": "Unknown molecular function",
  "gene": "UniProtKB:Q14183",
  "gene_name": "Double C2-like domain-containing protein alpha"
}